{
  "gene_name": "Cytosolic endo-beta-N-acetylglucosaminidase",
  "term_label": "Unknown cellular component",
  "gene": "UniProtKB:Q8NFI3",
  "gene_symbol": "ENGASE",
  "term_id": "UNKNOWN:0003"
}